{
  "gene": "UniProtKB:Q9P273",
  "gene_symbol": "TENM3",
  "gene_name": "Teneurin-3",
  "term_id": "GO:0043005",
  "term_label": "neuron projection"
}